{
  "gene_name": "Histone-lysine N-methyltransferase SMYD1",
  "term_label": "histone H3K4 methyltransferase activity",
  "gene": "UniProtKB:Q8NB12",
  "term_id": "GO:0042800",
  "gene_symbol": "SMYD1"
}